aspartate-ammonia ligase activity [GO:0004071] (molecular function) Relationships: is a type of ammonia ligase activity [GO:0016211] Definition: Catalysis of the reaction: ATP + L-aspartate + NH3 = AMP + diphosphate + L-asparagine. Sources: EC:6.3.1.1 Also known as: L-asparagine synthetase activity, L-aspartate:ammonia ligase (AMP-forming), asparagine synthetase activity